thrombospondin complex [GO:1990341] (cellular component) Relationships: is a type of GO:0032991; BFO_0000050 extracellular matrix [GO:0031012] Definition: A homotrimeric or homopentameric glycoprotein that functions at the interface of the cell membrane and the extracellular matrix through its interactions with proteins and proteoglycans, such as collagens, integrins and fibronectin, to regulate matrix structure and cellular behaviour. References: PMID:18193164 Sources: GOC:bhm